mitochondrion to lysosome vesicle-mediated transport [GO:0099074] (biological process) Definition: Vesicle-mediated transport of cargo from the mitochondrion to the lysosome, mediated by a mitochondrion-derived vesicle. References: PMID:20619655 Sources: GOC:PARL-UCL, GOC:bc, GOC:pad Also known as: mitochondrion to lysosome transport Relationships: is a type of mitochondrial transport [GO:0006839]; is a type of lysosomal transport [GO:0007041]; is a type of mitochondrion-derived vesicle mediated transport [GO:0099075]